positive regulation of actin filament severing [GO:1903920] (biological process) Also known as: positive regulation of F-actin severing, up regulation of F-actin severing, up regulation of actin filament severing, up-regulation of F-actin severing, up-regulation of actin filament severing, upregulation of F-actin severing, upregulation of actin filament severing, activation of F-actin severing, activation of actin filament severing, activation of actin filament severing activity, activation of barbed-end actin capping/severing activity, positive regulation of actin filament severing activity, positive regulation of barbed-end actin capping/severing activity, up regulation of actin filament severing activity, up regulation of barbed-end actin capping/severing activity, up-regulation of actin filament severing activity, up-regulation of barbed-end actin capping/severing activity, upregulation of actin filament severing activity, upregulation of barbed-end actin capping/severing activity Definition: Any process that activates or increases the frequency, rate or extent of actin filament severing. References: PMID:23325791 Sources: GOC:TermGenie, GOC:als, GO_REF:0000058 Relationships: is a type of GO:0048522; is a type of regulation of actin filament severing [GO:1903918]; positively regulates actin filament severing [GO:0051014]